{
  "gene_name": "Immunoglobulin kappa variable 1-5",
  "gene": "UniProtKB:P01602",
  "term_id": "UNKNOWN:0001",
  "gene_symbol": "IGKV1-5",
  "term_label": "Unknown molecular function"
}